{
  "term_label": "Unknown molecular function",
  "gene_name": "Putative uncharacterized protein PRO1716",
  "term_id": "UNKNOWN:0001",
  "gene_symbol": "PRO1716",
  "gene": "UniProtKB:Q9UHU1"
}